tolerance induction [GO:0002507] (biological process) Definition: A process that directly activates any of the steps required for tolerance, a physiologic state in which the immune system does not react destructively against the components of an organism that harbors it or against antigens that are introduced to it. Subtypes: GO:0002249, tolerance induction dependent upon immune response [GO:0002461], central tolerance induction [GO:0002508], tolerance induction to self antigen [GO:0002513], B cell tolerance induction [GO:0002514], GO:0002517, natural killer cell tolerance induction [GO:0002519], macrophage tolerance induction [GO:0010931], tolerance induction to lipopolysaccharide [GO:0072573] Regulation: regulated by regulation of tolerance induction [GO:0002643]; negatively regulated by negative regulation of tolerance induction [GO:0002644]; positively regulated by positive regulation of tolerance induction [GO:0002645] Relationships: is_a GO:0002376; is part of immune system development [GO:0002520] Sources: GOC:jal, GO_REF:0000022, ISBN:0781735149